{
  "term_label": "replication fork processing",
  "gene_symbol": "FBH1",
  "gene_name": "F-box DNA helicase 1",
  "gene": "UniProtKB:Q8NFZ0",
  "term_id": "GO:0031297"
}